histone H3K36 acetyltransferase activity [GO:0044018] (molecular function) References: PMID:18552846 Definition: Catalysis of the reaction: acetyl-CoA + histone H3 L-lysine (position 36) = CoA + histone H3 N6-acetyl-L-lysine (position 36). Relationships: is a type of histone H3 acetyltransferase activity [GO:0010484] Note: Comment: Note that the residue position corresponds to the canonical human H3 histone (UniProtKB:P84243); this residue is conserved across all eukaryotes. Residue 1 is the first residue following removal of the initiating Methionine (Met). Note that each histone is encoded by multiple genes, and sequences may vary across different genes within an organism. Also known as: histone H3-K36 acetyltransferase activity, histone acetylase activity (H3-K36 specific), histone acetyltransferase activity (H3-K36 specific), histone lysine N-acetyltransferase activity (H3-K36 specific)